cell proliferation involved in metanephros development [GO:0072203] (biological process) Definition: The multiplication or reproduction of cells, resulting in the expansion of the population in the metanephros. Sources: GOC:mtg_kidney_jan10 Relationships: is a type of cell proliferation involved in kidney development [GO:0072111]; is part of metanephros development [GO:0001656] Subtypes: metanephric mesenchymal cell proliferation involved in metanephros development [GO:0072136], metanephric extraglomerular mesangial cell proliferation involved in metanephros development [GO:0072261], metanephric glomerular mesangial cell proliferation involved in metanephros development [GO:0072262], metanephric cap mesenchymal cell proliferation involved in metanephros development [GO:0090094]